{
  "term_label": "plasma membrane",
  "term_id": "GO:0005886",
  "gene_symbol": "KCNH1",
  "gene": "UniProtKB:O95259",
  "gene_name": "Potassium voltage-gated channel subfamily H member 1"
}